{
  "gene": "UniProtKB:Q7L311",
  "term_label": "Unknown molecular function",
  "gene_symbol": "ARMCX2",
  "gene_name": "Armadillo repeat-containing X-linked protein 2",
  "term_id": "UNKNOWN:0001"
}